8-oxo-dADP diphosphate phosphatase activity [GO:0102459] (molecular function) Sources: GOC:pz Also known as: 8-oxo-deoxyadenine diphosphate phosphatase activity Definition: Catalysis of the reaction: 8-oxo-dADP + H2O = 8-oxo-dAMP + hydrogenphosphate + H+. Relationships: is a type of GO:0017110